monocyte aggregation [GO:0070487] (biological process) References: PMID:12972508 Sources: GOC:sl Regulation: regulated by GO:1900623; negatively regulated by negative regulation of monocyte aggregation [GO:1900624]; positively regulated by positive regulation of monocyte aggregation [GO:1900625] Relationships: is a type of leukocyte aggregation [GO:0070486] Also known as: mononuclear phagocyte aggregation Definition: The adhesion of one monocyte to one or more other monocytes via adhesion molecules.